{
  "gene": "UniProtKB:Q86XQ3",
  "term_label": "voltage-gated calcium channel activity",
  "term_id": "GO:0005245",
  "gene_symbol": "CATSPER3",
  "gene_name": "Cation channel sperm-associated protein 3"
}